{
  "gene_symbol": "ST8SIA4",
  "term_label": "alpha-N-acetylneuraminate alpha-2,8-sialyltransferase activity",
  "gene": "UniProtKB:Q92187",
  "gene_name": "CMP-N-acetylneuraminate-poly-alpha-2,8-sialyltransferase",
  "term_id": "GO:0003828"
}